dolichyl-phosphate-mannose-protein mannosyltransferase Pmt5p-Pmt3p dimer complex [GO:0097585] (CC) References: PMID:12551906 Sources: GOC:jd Relationships: is a type of dolichyl-phosphate-mannose-protein mannosyltransferase complex [GO:0031502] Definition: A protein dimer complex that possesses dolichyl-phosphate-mannose-protein mannosyltransferase activity and, in S. cerevisiae, is composed of Pmt5p-Pmt3p. Also known as: Pmt5p-Pmt3p complex